{
  "term_id": "UNKNOWN:0002",
  "gene_name": "Small proline-rich protein 2G",
  "gene": "UniProtKB:Q9BYE4",
  "gene_symbol": "SPRR2G",
  "term_label": "Unknown biological process"
}